{
  "gene_name": "Zinc finger protein 324B",
  "gene": "UniProtKB:Q6AW86",
  "gene_symbol": "ZNF324B",
  "term_label": "regulation of transcription by RNA polymerase II",
  "term_id": "GO:0006357"
}